negative regulation of thymine transport [GO:0035366] (BP) Relationships: is a type of negative regulation of nucleobase-containing compound transport [GO:0032240]; is a type of regulation of thymine transport [GO:0035365]; negatively regulates thymine transport [GO:0035364] Definition: Any process that stops, prevents, or reduces the frequency, rate or extent of the directed movement of thymine, 5-methyluracil, into, out of or within a cell, or between cells, by means of some agent such as a transporter or pore. Sources: GOC:bf, GOC:sl Also known as: negative regulation of 5-methyluracil transport